{
  "term_id": "GO:0006355",
  "gene_symbol": "ZNF284",
  "term_label": "regulation of DNA-templated transcription",
  "gene": "UniProtKB:Q2VY69",
  "gene_name": "Zinc finger protein 284"
}